cytoskeletal motor inhibitor activity [GO:0140661] (molecular function) Also known as: motor activity inhibitor activity References: PMID:23142046 Relationships: is a type of cytoskeletal motor regulator activity [GO:0140659]; is a type of molecular function inhibitor activity [GO:0140678]; negatively regulates cytoskeletal motor activity [GO:0003774] Definition: Binds to and stops, prevents, or reduces the activity of a motor protein.